{
  "gene": "UniProtKB:P0CJ75",
  "term_label": "Unknown cellular component",
  "gene_symbol": "MTRNR2L8",
  "term_id": "UNKNOWN:0003",
  "gene_name": "Humanin-like 8"
}